mitotic chromosome condensation [GO:0007076] (BP) Subtypes: GO:1990892, mitotic chromosome centromere condensation [GO:1990893] Definition: The cell cycle process in which chromatin structure is compacted prior to and during mitosis in eukaryotic cells. Relationships: is a type of chromosome condensation [GO:0030261]; is a type of mitotic cell cycle process [GO:1903047]; is part of mitotic sister chromatid segregation [GO:0000070] Sources: GOC:mah, ISBN:0815316194 Regulation: regulated by regulation of mitotic chromosome condensation [GO:1903379]; positively regulated by GO:1903380; negatively regulated by negative regulation of mitotic chromosome condensation [GO:1905213]